{
  "term_id": "UNKNOWN:0002",
  "gene_name": "Transmembrane protein 128",
  "term_label": "Unknown biological process",
  "gene": "UniProtKB:Q5BJH2",
  "gene_symbol": "TMEM128"
}